regulation of calcium-mediated signaling [GO:0050848] (biological process) Definition: Any process that modulates the frequency, rate or extent of calcium-mediated signaling, the process in which a cell uses calcium ions to convert an extracellular signal into a response. Subtypes: negative regulation of calcium-mediated signaling [GO:0050849], positive regulation of calcium-mediated signaling [GO:0050850], GO:0106056, regulation of CAMKK-AMPK signaling cascade [GO:1905289] Also known as: regulation of calcium-mediated signalling Sources: GOC:ai Relationships: is a type of regulation of intracellular signal transduction [GO:1902531]; regulates calcium-mediated signaling [GO:0019722]